{
  "gene": "UniProtKB:Q5I7T1",
  "gene_name": "Putative Dol-P-Glc:Glc(2)Man(9)GlcNAc(2)-PP-Dol alpha-1,2-glucosyltransferase",
  "term_id": "GO:0106073",
  "gene_symbol": "ALG10B",
  "term_label": "dolichyl pyrophosphate Glc2Man9GlcNAc2 alpha-1,2-glucosyltransferase activity"
}